{
  "gene_symbol": "SLC7A9",
  "gene_name": "b(0,+)-type amino acid transporter 1",
  "gene": "UniProtKB:P82251",
  "term_id": "UNKNOWN:0003",
  "term_label": "Unknown cellular component"
}